large ribosomal subunit pre-assembly complex [GO:0140714] (CC) Relationships: is a type of protein folding chaperone complex [GO:0101031] Definition: A protein complex that assists early maturation of nascent 60S ribosomal subunits. The complex interacts with the large ribosomal subunit rRNA via one of the components (Urb2 in S. cerevisiae) and requires a RNA helicase (Dbp6 in S. cerevisiae). References: PMID:17145778, PMID:9528757 Sources: GOC:lnp